{
  "gene": "UniProtKB:Q9GZU3",
  "gene_name": "Transmembrane protein 39B",
  "gene_symbol": "TMEM39B",
  "term_label": "Unknown biological process",
  "term_id": "UNKNOWN:0002"
}